{
  "gene_name": "Uncharacterized protein C11orf96",
  "term_label": "Unknown cellular component",
  "gene_symbol": "C11orf96",
  "term_id": "UNKNOWN:0003",
  "gene": "UniProtKB:Q7Z7L8"
}